{
  "gene": "UniProtKB:Q96IR7",
  "term_id": "GO:0005739",
  "term_label": "mitochondrion",
  "gene_symbol": "HPDL",
  "gene_name": "4-hydroxyphenylpyruvate dioxygenase-like protein"
}